aggregation of unicellular organisms [GO:0098630] (biological process) Sources: GOC:dos Relationships: is a type of cell aggregation [GO:0098743] Also known as: aggregation of single cell organisms Subtypes: biofilm formation [GO:0042710] Definition: The clustering together of unicellular organisms in suspension form aggregates.